dGTP biosynthetic process from dGDP [GO:0006187] (biological process) Also known as: dGTP anabolism from dGDP, dGTP formation from dGDP, dGTP synthesis from dGDP Relationships: is a type of dGDP metabolic process [GO:0046066]; is a type of GO:0046071 Definition: The chemical reactions and pathways resulting in the formation of dGTP, deoxyguanosine triphosphate (2'-deoxyguanosine 5'-triphosphate) from other compounds, including gGDP, deoxyguanosine diphosphate. Sources: ISBN:0198506732